{
  "gene": "UniProtKB:Q92968",
  "term_label": "peroxisomal importomer complex",
  "gene_name": "Peroxisomal membrane protein PEX13",
  "term_id": "GO:1990429",
  "gene_symbol": "PEX13"
}